branched-chain amino acid metabolic process [GO:0009081] (biological process) Sources: GOC:ai Subtypes: isoleucine metabolic process [GO:0006549], GO:0006551, GO:0006573, GO:0009082, GO:0009083 Also known as: branched chain family amino acid metabolism Relationships: is a type of GO:0006520; is a type of carboxylic acid metabolic process [GO:0019752] Definition: The chemical reactions and pathways involving amino acids containing a branched carbon skeleton, comprising isoleucine, leucine and valine.